{
  "term_id": "GO:0031994",
  "gene": "UniProtKB:P18065",
  "gene_name": "Insulin-like growth factor-binding protein 2",
  "gene_symbol": "IGFBP2",
  "term_label": "insulin-like growth factor I binding"
}